symbiont-mediated suppression of host resistance gene-dependent defense response [GO:0033660] (biological process) Also known as: down regulation by symbiont of defense response in host by specific elicitors, down-regulation by symbiont of host gene-for-gene resistance, downregulation by symbiont of pathogen-race/host plant cultivar-specific resistance in symbiont, negative regulation by symbiont of host resistance gene-dependent defense response, suppression by symbiont of host resistance gene-dependent defense response, inhibition by symbiont of host resistance gene-dependent defense response Sources: GOC:pamgo_curators Definition: A process in which a symbiont inhibits or disrupts the normal execution of the resistance gene-dependent defense response of the host organism. The host is defined as the larger of the organisms involved in a symbiotic interaction. Relationships: is a type of symbiont-mediated suppression of host defenses [GO:0044414]; is a type of symbiont-mediated perturbation of host resistance gene-dependent defense response [GO:0052158]